embryonic heart tube formation [GO:0003144] (biological process) Subtypes: GO:0003145 Definition: The process that gives rise to the embryonic heart tube. This process pertains to the initial formation of a structure from unspecified parts. The embryonic heart tube is an epithelial tube that will give rise to the mature heart. Relationships: is a type of GO:0001838; is part of GO:0003143 Sources: GOC:mtg_heart